{
  "gene_name": "Pancreatic progenitor cell differentiation and proliferation factor-like protein",
  "gene_symbol": "PPDPFL",
  "gene": "UniProtKB:Q8WWR9",
  "term_id": "UNKNOWN:0001",
  "term_label": "Unknown molecular function"
}